{
  "gene_name": "Ribosome biogenesis protein BRX1 homolog",
  "term_label": "RNA binding",
  "gene": "UniProtKB:Q8TDN6",
  "term_id": "GO:0003723",
  "gene_symbol": "BRIX1"
}